{
  "gene_symbol": "ZSCAN2",
  "gene": "UniProtKB:Q7Z7L9",
  "gene_name": "Zinc finger and SCAN domain-containing protein 2",
  "term_label": "nucleus",
  "term_id": "GO:0005634"
}